{
  "term_id": "UNKNOWN:0001",
  "term_label": "Unknown molecular function",
  "gene_symbol": "NPTX2",
  "gene_name": "Neuronal pentraxin-2",
  "gene": "UniProtKB:P47972"
}